{
  "gene_name": "Keratin-associated protein 13-2",
  "gene_symbol": "KRTAP13-2",
  "term_id": "UNKNOWN:0002",
  "gene": "UniProtKB:Q52LG2",
  "term_label": "Unknown biological process"
}